leukotriene A4 biosynthetic process [GO:1901753] (biological process) Relationships: is a type of GO:0019370; is a type of long-chain fatty acid biosynthetic process [GO:0042759]; is a type of ether biosynthetic process [GO:1901503]; is a type of fatty acid derivative biosynthetic process [GO:1901570]; is a type of leukotriene A4 metabolic process [GO:1901751] References: PMID:23242647 Sources: GOC:TermGenie, GOC:yaf Also known as: LTA4 biosynthesis, eoxin A4 biosynthesis, leukotriene A4 anabolism, leukotriene A4 biosynthesis, leukotriene A4 formation, leukotriene A4 synthesis Definition: The chemical reactions and pathways resulting in the formation of leukotriene A4.